{
  "gene_name": "Isocitrate dehydrogenase [NADP] cytoplasmic",
  "gene": "UniProtKB:O75874",
  "term_id": "GO:0006102",
  "gene_symbol": "IDH1",
  "term_label": "isocitrate metabolic process"
}